{
  "term_id": "UNKNOWN:0002",
  "gene_name": "Oxidoreductase-like domain-containing protein 1",
  "term_label": "Unknown biological process",
  "gene": "UniProtKB:Q5BKU9",
  "gene_symbol": "OXLD1"
}